{
  "term_label": "Unknown molecular function",
  "term_id": "UNKNOWN:0001",
  "gene_symbol": "SOGA3",
  "gene": "UniProtKB:Q5TF21",
  "gene_name": "Protein SOGA3"
}